{
  "gene_name": "Arf-GAP with SH3 domain, ANK repeat and PH domain-containing protein 1",
  "term_label": "centriolar satellite",
  "gene_symbol": "ASAP1",
  "term_id": "GO:0034451",
  "gene": "UniProtKB:Q9ULH1"
}